peptidyl-L-3-oxoalanine biosynthetic process from peptidyl-cysteine or peptidyl-serine [GO:0018083] (biological process) Sources: RESID:AA0185 Definition: The modification of peptidyl-cysteine or peptidyl-serine to peptidyl-L-3-oxoalanine; characteristic of the active sites of arylsulfatases. Relationships: is a type of peptidyl-cysteine modification [GO:0018198]; is a type of peptidyl-serine modification [GO:0018209] Also known as: peptidyl-L-3-oxoalanine anabolism from peptidyl-cysteine or peptidyl-serine, peptidyl-L-3-oxoalanine formation from peptidyl-cysteine or peptidyl-serine, peptidyl-L-3-oxoalanine synthesis from peptidyl-cysteine or peptidyl-serine